{
  "gene": "UniProtKB:Q8TCQ1",
  "gene_symbol": "MARCHF1",
  "term_label": "early endosome membrane",
  "term_id": "GO:0031901",
  "gene_name": "E3 ubiquitin-protein ligase MARCHF1"
}